{
  "term_label": "autophagosome assembly",
  "gene_name": "Beclin-2",
  "gene": "UniProtKB:A8MW95",
  "term_id": "GO:0000045",
  "gene_symbol": "BECN2"
}